{
  "gene": "UniProtKB:Q96LI5",
  "gene_symbol": "CNOT6L",
  "term_id": "UNKNOWN:0003",
  "gene_name": "CCR4-NOT transcription complex subunit 6-like",
  "term_label": "Unknown cellular component"
}